{
  "gene": "UniProtKB:Q9UHR4",
  "gene_name": "Brain-specific angiogenesis inhibitor 1-associated protein 2-like protein 1",
  "gene_symbol": "BAIAP2L1",
  "term_label": "positive regulation of actin filament polymerization",
  "term_id": "GO:0030838"
}